{
  "term_id": "UNKNOWN:0001",
  "gene_symbol": "ZCWPW2",
  "term_label": "Unknown molecular function",
  "gene": "UniProtKB:Q504Y3",
  "gene_name": "Zinc finger CW-type PWWP domain protein 2"
}